{
  "term_label": "RNA polymerase II cis-regulatory region sequence-specific DNA binding",
  "gene_name": "Zinc finger protein with KRAB and SCAN domains 5",
  "gene_symbol": "ZKSCAN5",
  "gene": "UniProtKB:Q9Y2L8",
  "term_id": "GO:0000978"
}